orbitofrontal cortex development [GO:0021769] (biological process) Relationships: is a type of anatomical structure development [GO:0048856]; is part of GO:0021761 Sources: GOC:cls, GOC:dgh, GOC:dph, GOC:jid, GO_REF:0000021 Definition: The progression of the orbitofrontal cortex over time from its initial formation until its mature state. The orbitofrontal cortex is a cerebral cortex region located in the frontal lobe.